endocardial cell fate commitment [GO:0060957] (biological process) Definition: The commitment of a cell to an endocardial cell fate and its capacity to differentiate into an endocardial cell. An endocardial cell is a specialized endothelial cell that makes up the endocardium portion of the heart. Sources: GOC:mtg_heart Subtypes: GO:0061445 Relationships: is a type of GO:0060839; is a type of cardiac cell fate commitment [GO:0060911]; is part of endocardial cell differentiation [GO:0060956]